{
  "gene_name": "Nucleotide sugar transporter SLC35D1",
  "gene_symbol": "SLC35D1",
  "gene": "UniProtKB:Q9NTN3",
  "term_id": "GO:0015780",
  "term_label": "nucleotide-sugar transmembrane transport"
}